{
  "term_id": "GO:0006583",
  "gene_name": "Membrane-associated transporter protein",
  "term_label": "melanin biosynthetic process from tyrosine",
  "gene": "UniProtKB:Q9UMX9",
  "gene_symbol": "SLC45A2"
}